{
  "term_id": "GO:0005044",
  "gene_name": "Macrophage scavenger receptor types I and II",
  "gene": "UniProtKB:P21757",
  "term_label": "scavenger receptor activity",
  "gene_symbol": "MSR1"
}